establishment of RNA localization to telomere [GO:0097694] (biological process) References: PMID:26586433 Sources: GOC:BHF, GOC:BHF_telomere, GOC:rph Also known as: establishment of RNA localisation to telomere Relationships: is a type of GO:0051236 Regulation: regulated by regulation of establishment of RNA localization to telomere [GO:1904910]; negatively regulated by negative regulation of establishment of RNA localization to telomere [GO:1904911]; positively regulated by positive regulation of establishment of RNA localization to telomere [GO:1904912] Definition: The directed movement of RNA to a specific location in the telomeric region of a chromosome.